{
  "term_label": "cell-cell signaling",
  "gene_symbol": "GJB1",
  "term_id": "GO:0007267",
  "gene_name": "Gap junction beta-1 protein",
  "gene": "UniProtKB:P08034"
}